negative regulation of mitochondrial DNA metabolic process [GO:1901859] (biological process) References: PMID:23150719 Sources: GOC:TermGenie, GOC:yaf Definition: Any process that stops, prevents or reduces the frequency, rate or extent of mitochondrial DNA metabolic process. Also known as: down regulation of mitochondrial DNA metabolic process, down regulation of mitochondrial DNA metabolism, down regulation of mtDNA metabolic process, down regulation of mtDNA metabolism, down-regulation of mitochondrial DNA metabolic process, down-regulation of mitochondrial DNA metabolism, down-regulation of mtDNA metabolic process, down-regulation of mtDNA metabolism, downregulation of mitochondrial DNA metabolic process, downregulation of mitochondrial DNA metabolism, downregulation of mtDNA metabolic process, downregulation of mtDNA metabolism, inhibition of mitochondrial DNA metabolism, inhibition of mtDNA metabolic process, inhibition of mtDNA metabolism, negative regulation of mitochondrial DNA metabolism, negative regulation of mtDNA metabolic process, negative regulation of mtDNA metabolism, inhibition of mitochondrial DNA metabolic process Subtypes: negative regulation of mitochondrial DNA replication [GO:0090298] Relationships: is a type of negative regulation of DNA metabolic process [GO:0051053]; is_a regulation of mitochondrial DNA metabolic process [GO:1901858]; negatively regulates mitochondrial DNA metabolic process [GO:0032042]